{
  "gene_name": "Zinc finger protein 716",
  "term_id": "GO:0000978",
  "gene_symbol": "ZNF716",
  "gene": "UniProtKB:A6NP11",
  "term_label": "RNA polymerase II cis-regulatory region sequence-specific DNA binding"
}